detection of chemical stimulus involved in sensory perception [GO:0050907] (biological process) Sources: GOC:ai, GOC:dos Definition: The series of events in which a chemical stimulus is received and converted into a molecular signal as part of sensory perception. Subtypes: detection of chemical stimulus involved in sensory perception of smell [GO:0050911], detection of chemical stimulus involved in sensory perception of taste [GO:0050912], GO:0050968, GO:0050969 Also known as: sensory detection of chemical stimulus, sensory detection of chemical stimulus during sensory perception, sensory perception, sensory detection of chemical stimulus, sensory perception, sensory transduction of chemical stimulus, sensory transduction of chemical stimulus, sensory transduction of chemical stimulus during sensory perception Relationships: is a type of detection of chemical stimulus [GO:0009593]; is a type of detection of stimulus involved in sensory perception [GO:0050906]; is part of GO:0007606